regulation of phosphatidylinositol biosynthetic process [GO:0010511] (biological process) Definition: Any process that modulates the frequency, rate or extent of the chemical reactions and pathways resulting in the formation of phosphatidylinositol. Sources: GOC:dph, GOC:tb, GOC:vw Relationships: is a type of regulation of phospholipid biosynthetic process [GO:0071071]; regulates GO:0006661 Subtypes: negative regulation of phosphatidylinositol biosynthetic process [GO:0010512], positive regulation of phosphatidylinositol biosynthetic process [GO:0010513], regulation of 1-phosphatidyl-1D-myo-inositol 4,5-bisphosphate biosynthetic process [GO:1902646]